{
  "term_label": "cytoplasm",
  "gene_name": "Adenosine deaminase domain-containing protein 1",
  "term_id": "GO:0005737",
  "gene_symbol": "ADAD1",
  "gene": "UniProtKB:Q96M93"
}